innate vocalization behavior [GO:0098582] (biological process) Relationships: is a type of vocalization behavior [GO:0071625] Definition: A vocalisation behavior that is innate, i.e. that does not need to be learned in order to occur. Sources: GOC:BHF, GOC:dos, GOC:rl